{
  "gene_symbol": "MYLK2",
  "term_label": "myosin light chain binding",
  "gene": "UniProtKB:Q9H1R3",
  "term_id": "GO:0032027",
  "gene_name": "Myosin light chain kinase 2, skeletal_cardiac muscle"
}